{
  "gene_symbol": "SEMA3E",
  "term_id": "GO:0001755",
  "gene_name": "Semaphorin-3E",
  "term_label": "neural crest cell migration",
  "gene": "UniProtKB:O15041"
}